melanocyte differentiation [GO:0030318] (biological process) Subtypes: early stripe melanocyte differentiation [GO:0050933], late stripe melanocyte differentiation [GO:0050934] Definition: The process in which a relatively unspecialized cell acquires specialized features of a melanocyte. Also known as: melanocyte cell differentiation, melanophore differentiation Regulation: regulated by regulation of melanocyte differentiation [GO:0045634]; negatively regulated by negative regulation of melanocyte differentiation [GO:0045635]; positively regulated by positive regulation of melanocyte differentiation [GO:0045636] Sources: GOC:mah Relationships: is a type of pigment cell differentiation [GO:0050931]